{
  "gene": "UniProtKB:P17019",
  "term_id": "GO:0000978",
  "gene_name": "Zinc finger protein 708",
  "gene_symbol": "ZNF708",
  "term_label": "RNA polymerase II cis-regulatory region sequence-specific DNA binding"
}